amylase activity [GO:0016160] (molecular function) Subtypes: GO:0004556, beta-amylase activity [GO:0016161] Definition: Catalysis of the hydrolysis of amylose or an amylose derivative. Relationships: is a type of GO:0004553 Sources: GOC:ai